protein phosphorylation [GO:0006468] (biological process) Regulation: regulated by regulation of protein phosphorylation [GO:0001932]; negatively regulated by negative regulation of protein phosphorylation [GO:0001933]; positively regulated by GO:0001934 Sources: GOC:hb Also known as: protein amino acid phosphorylation Relationships: is a type of phosphorylation [GO:0016310]; is a type of GO:0036211 Definition: The process of introducing a phosphate group on to a protein. Subtypes: inhibitory G protein-coupled receptor phosphorylation [GO:0002030], I-kappaB phosphorylation [GO:0007252], JUN phosphorylation [GO:0007258], GO:0010998, peptidyl-serine phosphorylation [GO:0018105], GO:0018106, peptidyl-threonine phosphorylation [GO:0018107], peptidyl-tyrosine phosphorylation [GO:0018108], peptidyl-arginine phosphorylation [GO:0018109], GO:0018217, GO:0046777